cytoplasmic capsid assembly [GO:0039709] (biological process) Sources: VZ:1950 Relationships: is a type of GO:0019069; occurs in host cell cytoplasm [GO:0030430] Subtypes: cytoplasmic icosahedral capsid assembly [GO:0039710], GO:0039711 Definition: The assembly of a virus capsid that occurs in the cytoplasm.